dinucleotide phosphatase activity [GO:0004551] (molecular function) Relationships: is_a pyrophosphatase activity [GO:0016462] Also known as: nucleotide diphosphatase activity, nucleotide pyrophosphatase activity, dinucleotide nucleotidohydrolase activity Subtypes: NAD+ diphosphatase activity [GO:0000210], NADPH pyrophosphatase activity [GO:0010943], NADH pyrophosphatase activity [GO:0035529], GO:0047884 References: PMID:2848456, PMID:4405504 Definition: Catalysis of the reaction: a dinucleotide + H2O = 2 mononucleotides.